{
  "gene_symbol": "OR1L3",
  "term_label": "plasma membrane",
  "gene": "UniProtKB:Q8NH93",
  "term_id": "GO:0005886",
  "gene_name": "Olfactory receptor 1L3"
}